{
  "term_id": "UNKNOWN:0003",
  "gene_symbol": "DPH5",
  "gene_name": "Diphthine methyl ester synthase",
  "term_label": "Unknown cellular component",
  "gene": "UniProtKB:Q9H2P9"
}